response to interleukin-8 [GO:0098758] (biological process) Definition: Any process that results in a change in state or activity of a cell or an organism (in terms of movement, secretion, enzyme production, gene expression, etc.) as a result of an interleukin-8 stimulus. Also known as: response to IL-8 Relationships: is a type of response to cytokine [GO:0034097] Subtypes: GO:0098759 Sources: GOC:BHF, GOC:mah